{
  "term_id": "UNKNOWN:0001",
  "gene_symbol": "VPS26C",
  "term_label": "Unknown molecular function",
  "gene_name": "Vacuolar protein sorting-associated protein 26C",
  "gene": "UniProtKB:O14972"
}